{
  "term_label": "positive regulation of mitochondrial fission",
  "gene_name": "Mitochondrial fission factor",
  "gene_symbol": "MFF",
  "term_id": "GO:0090141",
  "gene": "UniProtKB:Q9GZY8"
}